{
  "gene_symbol": "NOMO3",
  "term_id": "UNKNOWN:0001",
  "gene": "UniProtKB:P69849",
  "term_label": "Unknown molecular function",
  "gene_name": "BOS complex subunit NOMO3"
}